post-Golgi vesicle-mediated transport [GO:0006892] (biological process) Relationships: is a type of GO:0048193 Sources: GOC:ai, GOC:mah Also known as: post-Golgi transport Subtypes: GO:0006893, GO:0006895, GO:0006896 Definition: The directed movement of substances from the Golgi to other parts of the cell, including organelles and the plasma membrane, mediated by small transport vesicles.